cardiac neural crest cell development involved in outflow tract morphogenesis [GO:0061309] (biological process) Definition: The process aimed at the progression of a cardiac neural crest cell over time, from initial commitment of the cell to its specific fate, to the fully functional differentiated cell that contributes to the shaping of the outflow tract. Sources: GOC:dph, GOC:mtg_heart Relationships: is a type of cardiac neural crest cell development involved in heart development [GO:0061308]; is part of outflow tract morphogenesis [GO:0003151]